ligase activity, forming carbon-oxygen bonds [GO:0016875] (molecular function) Definition: Catalysis of the joining of two molecules via a carbon-oxygen bond, with the concomitant hydrolysis of the diphosphate bond in ATP or a similar triphosphate. Subtypes: GO:0004812, D-alanine-(R)-lactate ligase activity [GO:0160220] Relationships: is_a GO:0016874 Sources: EC:6.1.-.-